{
  "gene_symbol": "OR10H2",
  "term_id": "GO:0005886",
  "term_label": "plasma membrane",
  "gene": "UniProtKB:O60403",
  "gene_name": "Olfactory receptor 10H2"
}